{
  "gene_symbol": "RHPN1",
  "gene": "UniProtKB:Q8TCX5",
  "term_id": "UNKNOWN:0001",
  "gene_name": "Rhophilin-1",
  "term_label": "Unknown molecular function"
}